{
  "gene": "UniProtKB:O00238",
  "gene_name": "Bone morphogenetic protein receptor type-1B",
  "gene_symbol": "BMPR1B",
  "term_id": "GO:0071363",
  "term_label": "cellular response to growth factor stimulus"
}